{
  "gene_symbol": "USP12",
  "term_id": "GO:0005634",
  "gene": "UniProtKB:O75317",
  "term_label": "nucleus",
  "gene_name": "Ubiquitin carboxyl-terminal hydrolase 12"
}